senescence-associated vacuole [GO:0010282] (cellular component) Definition: A lytic vacuole that is maintained at acidic pH and has different tonoplast composition compared to the central vacuole. Found during leaf senescence and develops in the peripheral cytoplasm of cells that contain chloroplast. References: PMID:15743448 Relationships: is a type of lytic vacuole [GO:0000323]; is a type of plant-type vacuole [GO:0000325] Also known as: senescence associated vacuole